{
  "term_label": "RNA polymerase II transcription regulatory region sequence-specific DNA binding",
  "gene_name": "Zinc finger protein 558",
  "gene_symbol": "ZNF558",
  "term_id": "GO:0000977",
  "gene": "UniProtKB:Q96NG5"
}